homocysteine catabolic process [GO:0043418] (biological process) Definition: The chemical reactions and pathways resulting in the breakdown of homocysteine, the amino acid alpha-amino-gamma-mercaptobutanoic acid. Relationships: is a type of GO:0000098; is_a GO:0050667; is a type of non-proteinogenic amino acid catabolic process [GO:0170044]; is a type of GO:1901606 Also known as: homocysteine breakdown, homocysteine catabolism, homocysteine degradation Sources: GOC:jl